{
  "term_id": "UNKNOWN:0001",
  "gene_symbol": "DTWD2",
  "gene_name": "tRNA-uridine aminocarboxypropyltransferase 2",
  "term_label": "Unknown molecular function",
  "gene": "UniProtKB:Q8NBA8"
}